{
  "gene_symbol": "SRR",
  "gene_name": "Serine racemase",
  "term_label": "magnesium ion binding",
  "term_id": "GO:0000287",
  "gene": "UniProtKB:Q9GZT4"
}